{
  "gene_symbol": "NEK4",
  "term_label": "regulation of monoatomic cation transmembrane transport",
  "gene_name": "Serine_threonine-protein kinase Nek4",
  "term_id": "GO:1904062",
  "gene": "UniProtKB:P51957"
}